{
  "gene": "UniProtKB:Q14525",
  "gene_symbol": "KRT33B",
  "term_label": "morphogenesis of an epithelium",
  "gene_name": "Keratin, type I cuticular Ha3-II",
  "term_id": "GO:0002009"
}